{
  "term_id": "UNKNOWN:0001",
  "gene_symbol": "TNFRSF8",
  "gene_name": "Tumor necrosis factor receptor superfamily member 8",
  "gene": "UniProtKB:P28908",
  "term_label": "Unknown molecular function"
}